{
  "term_id": "GO:0009887",
  "gene": "UniProtKB:P40424",
  "gene_name": "Pre-B-cell leukemia transcription factor 1",
  "gene_symbol": "PBX1",
  "term_label": "animal organ morphogenesis"
}